{
  "gene": "UniProtKB:A0A075B6V1",
  "term_label": "Unknown biological process",
  "gene_name": "T cell receptor alpha joining 43 (Fragment)",
  "gene_symbol": "TRAJ43",
  "term_id": "UNKNOWN:0002"
}